{
  "gene": "UniProtKB:B5ME19",
  "gene_symbol": "EIF3CL",
  "term_id": "GO:0031369",
  "term_label": "translation initiation factor binding",
  "gene_name": "Eukaryotic translation initiation factor 3 subunit C-like protein"
}